pancreas induction [GO:0061132] (biological process) Sources: GOC:dph Definition: The close range interaction of two or more cells or tissues that causes the cells of the gut to change their fates and specify the development of the pancreas. Relationships: is a type of organ induction [GO:0001759]; is a type of regulation of morphogenesis of a branching structure [GO:0060688]; is a type of positive regulation of epithelial tube formation [GO:1905278]; RO_0002213 pancreas field specification [GO:0061131]